S-methyl-5-thioribose kinase activity [GO:0046522] (molecular function) Relationships: is a type of kinase activity [GO:0016301]; is a type of phosphotransferase activity, alcohol group as acceptor [GO:0016773] Also known as: 5-methylthioribose kinase activity, 5-methylthioribose kinase (phosphorylating), ATP:S-methyl-5-thio-D-ribose 1-phosphotransferase activity, ATP:S5-methyl-5-thio-D-ribose 1-phosphotransferase activity, MTR kinase activity, methylthioribose kinase activity Definition: Catalysis of the reaction: S-methyl-5-thio-D-ribose + ATP = S-methyl-5-thio-alpha-D-ribose 1-phosphate + ADP + 2 H+. Sources: EC:2.7.1.100, RHEA:22312